positive regulation of response to salt stress [GO:1901002] (biological process) Also known as: activation of response to ionic osmotic stress, activation of salinity response, positive regulation of response to ionic osmotic stress, positive regulation of salinity response, up regulation of response to ionic osmotic stress, up regulation of response to salt stress, up regulation of salinity response, up-regulation of response to ionic osmotic stress, up-regulation of response to salt stress, up-regulation of salinity response, upregulation of response to ionic osmotic stress, upregulation of response to salt stress, upregulation of salinity response, activation of response to salt stress Definition: Any process that activates or increases the frequency, rate or extent of response to salt stress. Relationships: is a type of GO:0048584; is_a regulation of response to salt stress [GO:1901000]; positively regulates response to salt stress [GO:0009651] References: PMID:22627139 Sources: GOC:TermGenie